shikimate O-hydroxycinnamoyltransferase activity [GO:0047172] (molecular function) Definition: Catalysis of the reaction: shikimate + coumaroyl-CoA = 4-coumaroylshikimate + CoA. Sources: EC:2.3.1.133, MetaCyc:2.3.1.133-RXN Also known as: 4-coumaroyl-CoA:shikimate O-(hydroxycinnamoyl)transferase activity, shikimate hydroxycinnamoyltransferase activity Relationships: is a type of O-hydroxycinnamoyltransferase activity [GO:0050737]